{
  "gene_name": "Neurogenic locus notch homolog protein 4",
  "term_id": "UNKNOWN:0002",
  "term_label": "Unknown biological process",
  "gene_symbol": "NOTCH4",
  "gene": "UniProtKB:Q99466"
}